{
  "term_label": "neuronal cell body",
  "gene": "UniProtKB:P01210",
  "gene_name": "Proenkephalin-A",
  "gene_symbol": "PENK",
  "term_id": "GO:0043025"
}